{
  "term_label": "GPI anchor biosynthetic process",
  "gene_symbol": "PIGH",
  "gene": "UniProtKB:Q14442",
  "term_id": "GO:0006506",
  "gene_name": "Phosphatidylinositol N-acetylglucosaminyltransferase subunit H"
}